{
  "gene": "UniProtKB:Q5KU26",
  "term_id": "GO:0006910",
  "gene_symbol": "COLEC12",
  "term_label": "phagocytosis, recognition",
  "gene_name": "Collectin-12"
}